biotinidase activity [GO:0047708] (molecular function) Sources: EC:3.5.1.12, MetaCyc:BIOTINIDASE-RXN Also known as: amidohydrolase biotinidase activity, biotin-amide amidohydrolase activity Definition: Catalysis of the reaction: biotin amide + H2O = biotin + NH3. Relationships: is a type of hydrolase activity, acting on carbon-nitrogen (but not peptide) bonds, in linear amides [GO:0016811]